{
  "gene": "UniProtKB:Q9NYQ8",
  "term_id": "UNKNOWN:0001",
  "term_label": "Unknown molecular function",
  "gene_name": "Protocadherin Fat 2",
  "gene_symbol": "FAT2"
}